{
  "gene": "UniProtKB:Q86W92",
  "gene_symbol": "PPFIBP1",
  "term_label": "presynaptic active zone",
  "gene_name": "Liprin-beta-1",
  "term_id": "GO:0048786"
}